{
  "gene": "UniProtKB:Q9H5H4",
  "term_label": "nucleus",
  "term_id": "GO:0005634",
  "gene_name": "Zinc finger protein 768",
  "gene_symbol": "ZNF768"
}